positive regulation of metanephric podocyte development [GO:2000478] (biological process) Also known as: positive regulation of metanephric glomerular visceral epithelial cell development Sources: GOC:obol Relationships: is a type of positive regulation of cell development [GO:0010720]; is a type of GO:2000477; positively regulates GO:0072249 Definition: Any process that activates or increases the frequency, rate or extent of metanephric glomerular visceral epithelial cell development.